{
  "term_id": "GO:0001640",
  "term_label": "adenylate cyclase inhibiting G protein-coupled glutamate receptor activity",
  "gene": "UniProtKB:Q14833",
  "gene_name": "Metabotropic glutamate receptor 4",
  "gene_symbol": "GRM4"
}